lipoprotein particle receptor binding [GO:0070325] (molecular function) Subtypes: low-density lipoprotein particle receptor binding [GO:0050750], GO:0070326, high-density lipoprotein particle receptor binding [GO:0070653] Definition: Binding to a lipoprotein particle receptor. Sources: GOC:BHF, GOC:rl Relationships: is a type of signaling receptor binding [GO:0005102]